{
  "term_id": "GO:1902895",
  "gene_name": "Endothelial transcription factor GATA-2",
  "gene_symbol": "GATA2",
  "gene": "UniProtKB:P23769",
  "term_label": "positive regulation of miRNA transcription"
}